{
  "gene_symbol": "ARHGAP1",
  "gene_name": "Rho GTPase-activating protein 1",
  "term_id": "GO:0007264",
  "gene": "UniProtKB:Q07960",
  "term_label": "small GTPase-mediated signal transduction"
}